{
  "term_id": "GO:0004148",
  "gene_symbol": "DLD",
  "gene_name": "Dihydrolipoyl dehydrogenase, mitochondrial",
  "gene": "UniProtKB:P09622",
  "term_label": "dihydrolipoyl dehydrogenase (NADH) activity"
}